{
  "gene": "UniProtKB:O76064",
  "term_label": "nucleus",
  "gene_symbol": "RNF8",
  "term_id": "GO:0005634",
  "gene_name": "E3 ubiquitin-protein ligase RNF8"
}